{
  "term_id": "GO:0019221",
  "term_label": "cytokine-mediated signaling pathway",
  "gene_name": "Leukocyte immunoglobulin-like receptor subfamily B member 4",
  "gene_symbol": "LILRB4",
  "gene": "UniProtKB:Q8NHJ6"
}